{
  "gene_symbol": "MFAP4",
  "gene": "UniProtKB:P55083",
  "term_id": "UNKNOWN:0001",
  "gene_name": "Microfibril-associated glycoprotein 4",
  "term_label": "Unknown molecular function"
}